{
  "term_id": "GO:0036502",
  "gene_name": "Selenoprotein S",
  "term_label": "Derlin-1-VIMP complex",
  "gene_symbol": "SELENOS",
  "gene": "UniProtKB:Q9BQE4"
}